{
  "gene_name": "FMR1-interacting protein NUFIP1",
  "term_id": "GO:0005634",
  "gene": "UniProtKB:Q9UHK0",
  "gene_symbol": "NUFIP1",
  "term_label": "nucleus"
}